{
  "gene_symbol": "MAP1LC3C",
  "term_label": "autophagosome maturation",
  "gene": "UniProtKB:Q9BXW4",
  "gene_name": "Microtubule-associated proteins 1A_1B light chain 3C",
  "term_id": "GO:0097352"
}